torso binding [GO:0005122] (molecular function) References: PMID:2927509 Sources: GOC:ceb Definition: Binding to a torso (tor) protein, a receptor tyrosine kinase. Also known as: tor binding, tor ligand, torso ligand Relationships: is a type of GO:0005102